{
  "term_label": "endocytic recycling",
  "gene_name": "WASH complex subunit 1",
  "term_id": "GO:0032456",
  "gene": "UniProtKB:A8K0Z3",
  "gene_symbol": "WASHC1"
}